{
  "gene_name": "Sentan",
  "term_id": "GO:0005509",
  "gene_symbol": "SNTN",
  "gene": "UniProtKB:A6NMZ2",
  "term_label": "calcium ion binding"
}